{
  "term_id": "GO:0005886",
  "gene": "UniProtKB:Q9NTN9",
  "gene_symbol": "SEMA4G",
  "gene_name": "Semaphorin-4G",
  "term_label": "plasma membrane"
}